{
  "term_id": "UNKNOWN:0002",
  "term_label": "Unknown biological process",
  "gene": "UniProtKB:Q92583",
  "gene_name": "C-C motif chemokine 17",
  "gene_symbol": "CCL17"
}